{
  "gene_symbol": "FOXF2",
  "gene": "UniProtKB:Q12947",
  "term_label": "nucleus",
  "term_id": "GO:0005634",
  "gene_name": "Forkhead box protein F2"
}